{
  "gene_symbol": "SHMT2",
  "term_label": "glycine hydroxymethyltransferase activity",
  "gene": "UniProtKB:P34897",
  "gene_name": "Serine hydroxymethyltransferase, mitochondrial",
  "term_id": "GO:0004372"
}